{
  "gene_symbol": "CD48",
  "gene": "UniProtKB:P09326",
  "term_label": "Unknown molecular function",
  "term_id": "UNKNOWN:0001",
  "gene_name": "CD48 antigen"
}